{
  "gene": "UniProtKB:Q13510",
  "gene_symbol": "ASAH1",
  "gene_name": "Acid ceramidase",
  "term_label": "Unknown cellular component",
  "term_id": "UNKNOWN:0003"
}